{
  "gene": "UniProtKB:P07203",
  "gene_symbol": "GPX1",
  "term_id": "GO:0042744",
  "term_label": "hydrogen peroxide catabolic process",
  "gene_name": "Glutathione peroxidase 1"
}